cellular stress response to acid chemical [GO:0097533] (biological process) Definition: Any process that results in a change in state or activity of a cell (in terms of movement, secretion, enzyme production, gene expression, etc.) as a result of a disturbance in cellular homeostasis caused by the chemical structure of the anion portion of a dissociated acid (rather than the acid acting as a proton donor). The acid chemical may be in gaseous, liquid or solid form. References: PMID:10615049, PMID:19170886 Sources: GOC:BHF, GOC:aa, GOC:go_curators, GOC:rl, Wikipedia:Acid Relationships: is a type of stress response to acid chemical [GO:0097532]; is part of cellular response to stress [GO:0033554]; is part of cellular response to acid chemical [GO:0071229] Also known as: cellular response to acid stress, cellular stress response to acid